L-tryptophan:2-oxoglutarate aminotransferase activity [GO:0050362] (molecular function) Definition: Catalysis of the reaction: L-tryptophan + 2-oxoglutarate = indolepyruvate + L-glutamate. Sources: EC:2.6.1.27, MetaCyc:TRYPTOPHAN-AMINOTRANSFERASE-RXN Also known as: L-tryptophan aminotransferase activity, L-tryptophan transaminase activity, tryptophan transaminase activity, tryptophan aminotransferase activity, 5-hydroxytryptophan-ketoglutaric transaminase activity, L-phenylalanine-2-oxoglutarate aminotransferase activity, hydroxytryptophan aminotransferase activity Relationships: is a type of L-tryptophan aminotransferase activity [GO:0070529]